{
  "gene_name": "Dual specificity protein kinase CLK4",
  "gene": "UniProtKB:Q9HAZ1",
  "term_id": "GO:0043484",
  "term_label": "regulation of RNA splicing",
  "gene_symbol": "CLK4"
}